ascus development [GO:0075317] (biological process) Relationships: is a type of GO:0075259 Note: Note that ascospores and asci are separate biological structures. The ascus is the structure that contain the ascospores, but the development of the ascus is a different process than the formation of the ascospores themselves; for instance, some mutations affect sporulation without affecting ascus development. For this reason, GO:0030437 ascospore formation and GO:0075317 ascus development are different terms and are not linked. Sources: GOC:di, GOC:mah, GOC:mcc, GOC:pamgo_curators Definition: The process that leads to the development of ascus, a sac-like structure produced by fungi of the phylum Ascomycota (sac fungi) in which sexually produced spores (ascospores), usually four or eight in number, are formed. Regulation: regulated by regulation of ascus development [GO:0075318]; positively regulated by GO:0075319; negatively regulated by negative regulation of ascus development [GO:0075320]